{
  "gene": "UniProtKB:Q9UBS3",
  "gene_symbol": "DNAJB9",
  "gene_name": "DnaJ homolog subfamily B member 9",
  "term_id": "GO:0051787",
  "term_label": "misfolded protein binding"
}